phosphatidylglycerol dehydrogenase (NAD+) activity [GO:0160242] (molecular function) Definition: Catalysis of the reaction: a 1,2-diacyl-sn-glycero-3-phospho-(1'-sn-glycerol) + NAD+ = a 1,2-diacyl-sn-glycero-3-phospho-(1'-sn-glycerone) + NADH + H+. References: PMID:26338420 Sources: RHEA:81099 Relationships: is a type of oxidoreductase activity, acting on the CH-OH group of donors, NAD or NADP as acceptor [GO:0016616]